{
  "term_id": "GO:1902531",
  "gene_name": "Ras GTPase-activating protein 2",
  "gene_symbol": "RASA2",
  "term_label": "regulation of intracellular signal transduction",
  "gene": "UniProtKB:Q15283"
}